{
  "term_label": "plasma membrane",
  "term_id": "GO:0005886",
  "gene": "UniProtKB:Q16720",
  "gene_name": "Plasma membrane calcium-transporting ATPase 3",
  "gene_symbol": "ATP2B3"
}